{
  "gene_name": "Diacylglycerol kinase gamma",
  "gene_symbol": "DGKG",
  "term_label": "diacylglycerol metabolic process",
  "term_id": "GO:0046339",
  "gene": "UniProtKB:P49619"
}